{
  "term_id": "GO:0005737",
  "gene_name": "Ferroptosis suppressor protein 1",
  "gene": "UniProtKB:Q9BRQ8",
  "term_label": "cytoplasm",
  "gene_symbol": "AIFM2"
}